{
  "term_label": "olfactory receptor activity",
  "gene_name": "Olfactory receptor 52N5",
  "gene_symbol": "OR52N5",
  "term_id": "GO:0004984",
  "gene": "UniProtKB:Q8NH56"
}